{
  "gene_name": "Cysteine-rich PDZ-binding protein",
  "gene": "UniProtKB:Q9P021",
  "term_id": "GO:0031122",
  "gene_symbol": "CRIPT",
  "term_label": "cytoplasmic microtubule organization"
}